peptidyl-lysine 5-dioxygenase activity [GO:0070815] (molecular function) Also known as: lysine hydroxylase activity, lysine,2-oxoglutarate 5-dioxygenase activity, lysine-2-oxoglutarate dioxygenase activity, lysyl hydroxylase activity, peptide-lysine 5-dioxygenase activity, protein lysine hydroxylase activity, peptidyl-lysine, 2-oxoglutarate: oxygen oxidoreductase activity, peptidyllysine, 2-oxoglutarate:oxygen 5-oxidoreductase activity Definition: Catalysis of the reaction: L-lysyl-[protein] + 2-oxoglutarate + O2 = (5S)-5-hydroxy-L-lysyl-[protein] + succinate + CO2. Relationships: is a type of 2-oxoglutarate-dependent dioxygenase activity [GO:0016706]; is a type of catalytic activity, acting on a protein [GO:0140096] References: PMID:19574390 Sources: RHEA:58360